furaneol oxidoreductase activity [GO:0102978] (molecular function) Definition: Catalysis of the reaction: 4-hydroxy-2,5-dimethylfuran-3-one + NADP = 4-hydroxy-5-methyl-2-methylenefuran-3-one + NADPH + H+. Sources: EC:1.3.1.105, GOC:pz Relationships: is a type of oxidoreductase activity, acting on the CH-CH group of donors, NAD or NADP as acceptor [GO:0016628]